{
  "gene_name": "Glypican-4",
  "gene_symbol": "GPC4",
  "term_id": "GO:0009986",
  "term_label": "cell surface",
  "gene": "UniProtKB:O75487"
}